negative regulation of DNA binding [GO:0043392] (biological process) Subtypes: negative regulation of transcription regulatory region DNA binding [GO:2000678] Sources: GOC:dph, GOC:jl, GOC:tb Also known as: down regulation of DNA binding, down-regulation of DNA binding, downregulation of DNA binding, inhibition of DNA binding Relationships: is a type of negative regulation of binding [GO:0051100]; is a type of regulation of DNA binding [GO:0051101]; RO_0002212 DNA binding [GO:0003677] Definition: Any process that stops or reduces the frequency, rate or extent of DNA binding. DNA binding is any process in which a gene product interacts selectively with DNA (deoxyribonucleic acid).